endodeoxyribonuclease complex [GO:1905347] (cellular component) Definition: A protein complex which is capable of endodeoxyribonuclease activity. References: PMID:18413719 Sources: GOC:TermGenie, GOC:bhm, GO_REF:0000088 Also known as: Mus81-Eme1 complex, Mus81-Eme2 complex Note: An example of this is MUS81 in human (Q96NY9) in PMID:18413719 (inferred from direct assay). Relationships: is a type of endonuclease complex [GO:1905348] Subtypes: type II site-specific deoxyribonuclease complex [GO:0009359], excinuclease repair complex [GO:0009380], GO:0019812, type III site-specific deoxyribonuclease complex [GO:0019813], type IV site-specific deoxyribonuclease complex [GO:0032068], Holliday junction resolvase complex [GO:0048476]